{
  "term_id": "GO:0005783",
  "term_label": "endoplasmic reticulum",
  "gene_name": "17-beta-hydroxysteroid dehydrogenase type 3",
  "gene": "UniProtKB:P37058",
  "gene_symbol": "HSD17B3"
}